{
  "term_id": "GO:0005886",
  "gene_name": "XK-related protein 4",
  "gene_symbol": "XKR4",
  "term_label": "plasma membrane",
  "gene": "UniProtKB:Q5GH76"
}